{
  "term_label": "nucleus",
  "gene": "UniProtKB:A6NDZ8",
  "gene_symbol": "MBD3L4",
  "term_id": "GO:0005634",
  "gene_name": "Putative methyl-CpG-binding domain protein 3-like 4"
}